{
  "term_id": "UNKNOWN:0002",
  "gene_name": "Inactive ADP-ribosyltransferase ARH2",
  "gene_symbol": "ADPRHL1",
  "gene": "UniProtKB:Q8NDY3",
  "term_label": "Unknown biological process"
}